{
  "gene_symbol": "CADPS",
  "gene_name": "Calcium-dependent secretion activator 1",
  "gene": "UniProtKB:Q9ULU8",
  "term_id": "UNKNOWN:0001",
  "term_label": "Unknown molecular function"
}